radial spoke 2 [GO:0120334] (cellular component) Relationships: is a type of GO:0001534 Also known as: RS2 References: PMID:22754630 Sources: GOC:krc Definition: The radial spoke of each group of radial spokes, whether grouped as triplets or doublets, that is immediately distal to radial spoke 1 (RS1). Radial spoke 2 (RS2), similarly to RS1, is comprised of four domains: 1) a very short base anchored to the A microtubule, 2) an elongaged stalk, 3) a bifurcated neck, and 4) an orthogonal head. The base of RS2 is connected to the tail of the inner dynein arm c.